{
  "term_id": "GO:1902711",
  "gene": "UniProtKB:P34903",
  "term_label": "GABA-A receptor complex",
  "gene_name": "Gamma-aminobutyric acid receptor subunit alpha-3",
  "gene_symbol": "GABRA3"
}